mobile ion carrier activity [GO:0022809] (molecular function) Definition: Small molecule produced by bacteria that carries an ion across the membrane by enclosing the ion and travelling with the ion across the membrane. It does not form a fully open pore across the membrane. Sources: GOC:mtg_transport, GOC:pr, ISBN:0815340729 Relationships: is a type of transmembrane transporter activity [GO:0022857]; is part of monoatomic ion transmembrane transport [GO:0034220] Also known as: ionophore